{
  "gene_name": "Paternally-expressed gene 3 protein",
  "gene_symbol": "PEG3",
  "term_label": "DNA-binding transcription factor activity, RNA polymerase II-specific",
  "term_id": "GO:0000981",
  "gene": "UniProtKB:Q9GZU2"
}